{
  "gene_symbol": "ABO",
  "gene_name": "Histo-blood group ABO system transferase",
  "term_id": "GO:0005794",
  "term_label": "Golgi apparatus",
  "gene": "UniProtKB:P16442"
}